regulation of phospholipid efflux [GO:1902994] (biological process) Definition: Any process that modulates the frequency, rate or extent of phospholipid efflux. Subtypes: GO:1902995, GO:1902999 References: PMID:12042316 Sources: GOC:TermGenie, GOC:sjp, GO_REF:0000058 Relationships: is a type of GO:2001138; regulates phospholipid efflux [GO:0033700] Also known as: regulation of phospholipid export